{
  "term_id": "GO:0000149",
  "term_label": "SNARE binding",
  "gene": "UniProtKB:Q96JG6",
  "gene_name": "Syndetin",
  "gene_symbol": "VPS50"
}